{
  "gene": "UniProtKB:Q9BZE0",
  "term_id": "GO:0007417",
  "gene_symbol": "GLIS2",
  "gene_name": "Zinc finger protein GLIS2",
  "term_label": "central nervous system development"
}